{
  "gene_symbol": "CHMP4B",
  "term_id": "GO:0006900",
  "gene_name": "Charged multivesicular body protein 4b",
  "term_label": "vesicle budding from membrane",
  "gene": "UniProtKB:Q9H444"
}